{
  "gene": "UniProtKB:O60934",
  "term_id": "GO:0007095",
  "gene_symbol": "NBN",
  "gene_name": "Nibrin",
  "term_label": "mitotic G2 DNA damage checkpoint signaling"
}